{
  "gene_symbol": "NLRP3",
  "term_id": "GO:0050727",
  "gene": "UniProtKB:Q96P20",
  "gene_name": "NACHT, LRR and PYD domains-containing protein 3",
  "term_label": "regulation of inflammatory response"
}